{
  "gene": "UniProtKB:P55286",
  "gene_symbol": "CDH8",
  "term_id": "GO:0016342",
  "gene_name": "Cadherin-8",
  "term_label": "catenin complex"
}